{
  "gene": "UniProtKB:O95988",
  "term_label": "protein serine/threonine kinase activator activity",
  "gene_symbol": "TCL1B",
  "term_id": "GO:0043539",
  "gene_name": "T-cell leukemia_lymphoma protein 1B"
}